{
  "term_id": "GO:0030036",
  "term_label": "actin cytoskeleton organization",
  "gene": "UniProtKB:Q96JY6",
  "gene_name": "PDZ and LIM domain protein 2",
  "gene_symbol": "PDLIM2"
}